{
  "gene_symbol": "CDK13",
  "gene": "UniProtKB:Q14004",
  "term_id": "GO:0008353",
  "gene_name": "Cyclin-dependent kinase 13",
  "term_label": "RNA polymerase II CTD heptapeptide repeat kinase activity"
}